cilium movement involved in otolith formation [GO:0003355] (biological process) References: PMID:19043402 Sources: GOC:dph, GOC:krc Relationships: is a type of epithelial cilium movement involved in extracellular fluid movement [GO:0003351]; is part of otolith formation [GO:0032475] Definition: The directed, self-propelled movement of cilia of inner ear epithelial cells, resulting the aggregation of otolith seed particles.